mitochondrial double-strand break repair via homologous recombination [GO:0097552] (biological process) Definition: The repair of a double-strand break in mitochondrial DNA in which the broken DNA molecule is repaired using homologous sequences. References: PMID:22214610 Sources: GOC:di Also known as: mtDSB repair via homologous recombination Note: Note that the processes of nuclear double-strand break repair and mitochondrial double-strand break repair are genetically separable. Relationships: is a type of recombinational repair [GO:0000725]; is a type of mitochondrial double-strand break repair [GO:0097551]